{
  "gene": "UniProtKB:O00410",
  "term_label": "nuclear import signal receptor activity",
  "term_id": "GO:0061608",
  "gene_name": "Importin-5",
  "gene_symbol": "IPO5"
}